{
  "term_id": "GO:2000009",
  "term_label": "negative regulation of protein localization to cell surface",
  "gene": "UniProtKB:Q9HD26",
  "gene_name": "Golgi-associated PDZ and coiled-coil motif-containing protein",
  "gene_symbol": "GOPC"
}